{
  "term_label": "regulation of transcription by RNA polymerase II",
  "gene_symbol": "ZNF136",
  "gene_name": "Zinc finger protein 136",
  "gene": "UniProtKB:P52737",
  "term_id": "GO:0006357"
}